{
  "gene_symbol": "TMSB15A",
  "gene": "UniProtKB:P0CG34",
  "term_id": "GO:0003785",
  "gene_name": "Thymosin beta-15A",
  "term_label": "actin monomer binding"
}